{
  "gene": "UniProtKB:Q92643",
  "gene_symbol": "PIGK",
  "term_label": "GPI-anchor transamidase complex",
  "gene_name": "GPI-anchor transamidase",
  "term_id": "GO:0042765"
}